{
  "gene": "UniProtKB:Q7Z7K0",
  "term_id": "UNKNOWN:0002",
  "term_label": "Unknown biological process",
  "gene_name": "COX assembly mitochondrial protein homolog",
  "gene_symbol": "CMC1"
}